{
  "term_label": "protein export from nucleus",
  "gene_name": "Exportin-2",
  "term_id": "GO:0006611",
  "gene": "UniProtKB:P55060",
  "gene_symbol": "CSE1L"
}